{
  "gene_name": "Epithelial cell-transforming sequence 2 oncogene-like",
  "term_id": "UNKNOWN:0003",
  "gene_symbol": "ECT2L",
  "gene": "UniProtKB:Q008S8",
  "term_label": "Unknown cellular component"
}